adhesion of symbiont to host cell surface via host membrane carbohydrate [GO:0141024] (biological process) Relationships: is a type of adhesion of symbiont to host cell [GO:0044650] References: PMID:15210807, PMID:19527885, PMID:30736336 Definition: The attachment of a symbiont to its host by binding to a carbohydrate on the host cell surface. The host is defined as the larger of the organisms involved in a symbiotic interaction.